respiratory chain complex III [GO:0045275] (cellular component) Also known as: complex III, cytochrome bc(1) complex, cytochrome bc1 complex, ubiquinol-cytochrome c oxidoreductase complex, ubiquinol-cytochrome-c reductase complex, CoQH2-cytochrome c reductase complex, coenzyme Q-cytochrome c oxidoreductase complex, coenzyme Q-cytochrome c reductase complex, electron transport complex III Relationships: is a type of cytochrome complex [GO:0070069]; is a type of GO:0098803; is a type of transmembrane transporter complex [GO:1902495] References: PMID:16228398, PMID:16352458, PMID:17200733 Definition: A protein complex that transfers electrons from ubiquinol to cytochrome c and translocates two protons across a membrane. The complex contains a core structure of three catalytic subunits: cytochrome b, the Rieske iron sulfur protein (ISP), and cytochrome c1, which are arranged in an integral membrane-bound dimeric complex; additional subunits are present, and vary among different species.